snRNA modification [GO:0040031] (biological process) Subtypes: snRNA pseudouridine synthesis [GO:0031120], snRNA methylation [GO:0106349], snRNA (adenine-N6)-methylation [GO:0120049] Definition: The covalent alteration of one or more nucleotides within snRNA, resulting in a change in the properties of the snRNA. Relationships: is a type of RNA modification [GO:0009451]; is a type of snRNA processing [GO:0016180] Sources: GOC:jl